regulation of plasma membrane bounded cell projection assembly [GO:0120032] (biological process) Relationships: is a type of GO:0060491; is a type of regulation of plasma membrane bounded cell projection organization [GO:0120035]; regulates plasma membrane bounded cell projection assembly [GO:0120031] Definition: Any process that modulates the rate, frequency, or extent of plasma membrane bounded cell projection assembly. Subtypes: regulation of lamellipodium assembly [GO:0010591], regulation of pseudopodium assembly [GO:0031272], regulation of mating projection assembly [GO:0031383], regulation of microvillus assembly [GO:0032534], GO:0051489, negative regulation of plasma membrane bounded cell projection assembly [GO:0120033], GO:0120034, regulation of ruffle assembly [GO:1900027], regulation of cilium assembly [GO:1902017], regulation of bleb assembly [GO:1904170], GO:2000547 Sources: GOC:krc